{
  "gene_symbol": "OAS2",
  "gene": "UniProtKB:P29728",
  "term_id": "GO:0001730",
  "gene_name": "2'-5'-oligoadenylate synthase 2",
  "term_label": "2'-5'-oligoadenylate synthetase activity"
}